positive regulation of alkaline phosphatase activity [GO:0010694] (biological process) Relationships: is a type of positive regulation of phosphatase activity [GO:0010922]; positively regulates alkaline phosphatase activity [GO:0004035] Sources: GOC:dph, GOC:tb Definition: Any process that increases the frequency, rate or extent of alkaline phosphatase activity, the catalysis of the reaction: an orthophosphoric monoester + H2O = an alcohol + phosphate, with an alkaline pH optimum.